{
  "term_label": "GTPase activator activity",
  "gene_name": "TBC domain-containing protein kinase-like protein",
  "gene_symbol": "TBCK",
  "term_id": "GO:0005096",
  "gene": "UniProtKB:Q8TEA7"
}